{
  "gene": "UniProtKB:Q93079",
  "gene_name": "Histone H2B type 1-H",
  "term_id": "GO:0006325",
  "gene_symbol": "H2BC9",
  "term_label": "chromatin organization"
}